{
  "gene_symbol": "BRINP3",
  "gene_name": "BMP_retinoic acid-inducible neural-specific protein 3",
  "term_id": "GO:0071300",
  "gene": "UniProtKB:Q76B58",
  "term_label": "cellular response to retinoic acid"
}